gallate 1-beta-glucosyltransferase activity [GO:0047913] (molecular function) Sources: EC:2.4.1.136, RHEA:15249 Also known as: gallate 1-b-glucosyltransferase activity, UDP-glucose-vanillate 1-glucosyltransferase activity, UDP-glucose:gallate beta-D-glucosyltransferase activity, UDPglucose-vanillate 1-glucosyltransferase activity, UDPglucose:gallate beta-D-glucosyltransferase activity, UDPglucose:gallate glucosyltransferase activity, UDPglucose:vanillate 1-O-glucosyltransferase activity Relationships: is a type of UDP-glucosyltransferase activity [GO:0035251] Definition: Catalysis of the reaction: gallate + UDP-D-glucose = 1-O-galloyl-beta-D-glucose + UDP.